rRNA (uridine-N3-)-methyltransferase activity [GO:0070042] (molecular function) Definition: Catalysis of the reaction: S-adenosyl-L-methionine + rRNA = S-adenosyl-L-homocysteine + rRNA containing N3-methyluridine. Relationships: is_a N-methyltransferase activity [GO:0008170]; is a type of rRNA (uridine) methyltransferase activity [GO:0016436] Sources: GOC:imk, GOC:mah